{
  "gene_symbol": "CCT5",
  "term_id": "GO:0006457",
  "gene": "UniProtKB:P48643",
  "gene_name": "T-complex protein 1 subunit epsilon",
  "term_label": "protein folding"
}